{
  "gene_name": "Putative uncharacterized protein encoded by MIR7-3HG",
  "term_id": "UNKNOWN:0001",
  "gene_symbol": "MIR7-3HG",
  "term_label": "Unknown molecular function",
  "gene": "UniProtKB:Q8N6C7"
}